{
  "gene_symbol": "ATRAID",
  "gene": "UniProtKB:Q6UW56",
  "term_label": "Unknown cellular component",
  "gene_name": "All-trans retinoic acid-induced differentiation factor",
  "term_id": "UNKNOWN:0003"
}